negative regulation of neutrophil chemotaxis [GO:0090024] (biological process) Relationships: is a type of negative regulation of granulocyte chemotaxis [GO:0071623]; is_a GO:0090022; is_a GO:1902623; negatively regulates GO:0030593 Sources: GOC:dph, GOC:tb Definition: Any process that decreases the frequency, rate, or extent of neutrophil chemotaxis. Neutrophil chemotaxis is the directed movement of a neutrophil cell, the most numerous polymorphonuclear leukocyte found in the blood, in response to an external stimulus, usually an infection or wounding.